{
  "gene_symbol": "WDR19",
  "gene": "UniProtKB:Q8NEZ3",
  "term_label": "cilium",
  "term_id": "GO:0005929",
  "gene_name": "WD repeat-containing protein 19"
}